{
  "term_label": "tRNA binding",
  "gene": "UniProtKB:Q96Q11",
  "gene_name": "CCA tRNA nucleotidyltransferase 1, mitochondrial",
  "term_id": "GO:0000049",
  "gene_symbol": "TRNT1"
}